{
  "term_id": "UNKNOWN:0001",
  "term_label": "Unknown molecular function",
  "gene": "UniProtKB:Q8TAL6",
  "gene_symbol": "FIBIN",
  "gene_name": "Fin bud initiation factor homolog"
}